exoribonuclease complex [GO:1905354] (cellular component) Subtypes: GO:0000178, PAN complex [GO:0031251], GO:0045025, GO:0090730, GO:0110103 Note: An example of this is DIS3 in human (Q9Y2L1) in PMID:17174896 (inferred from direct assay). Relationships: is a type of GO:1902494 References: PMID:17174896 Sources: GOC:TermGenie, GOC:bhm, GO_REF:0000088 Definition: A protein complex which is capable of exoribonuclease activity.